{
  "gene_name": "Blood group Rh(CE) polypeptide",
  "term_label": "ammonium transmembrane transport",
  "gene": "UniProtKB:P18577",
  "term_id": "GO:0072488",
  "gene_symbol": "RHCE"
}